alpha-2 macroglobulin receptor activity [GO:0016964] (molecular function) Definition: Combining with alpha-2 macroglobulin and delivering alpha-2 macroglobulin into the cell via receptor-mediated endocytosis. Relationships: is a type of cargo receptor activity [GO:0038024] References: PMID:6188403 Sources: GOC:bf, GOC:ma